{
  "gene_symbol": "CASTOR2",
  "term_id": "UNKNOWN:0001",
  "term_label": "Unknown molecular function",
  "gene": "UniProtKB:A6NHX0",
  "gene_name": "Cytosolic arginine sensor for mTORC1 subunit 2"
}